RNA splicing, via transesterification reactions with bulged adenosine as nucleophile [GO:0000377] (BP) Definition: Splicing of RNA via a series of two transesterification reactions with a bulged adenosine residue from the intron branch point as the initiating nucleophile. When the initial RNA for the splicing reaction is a single molecule (cis splicing), the excised intron is released in a lariat structure. References: PMID:11377794 Sources: GOC:krc Also known as: lariat RNA biosynthesis, lariat RNA formation Relationships: is a type of GO:0000375 Subtypes: Group II intron splicing [GO:0000373], Group III intron splicing [GO:0000374], GO:0000398